{
  "term_label": "endocytosis",
  "term_id": "GO:0006897",
  "gene_symbol": "C9orf72",
  "gene": "UniProtKB:Q96LT7",
  "gene_name": "Guanine nucleotide exchange factor C9orf72"
}